{
  "gene": "UniProtKB:Q9UID3",
  "gene_name": "Vacuolar protein sorting-associated protein 51 homolog",
  "gene_symbol": "VPS51",
  "term_label": "EARP complex",
  "term_id": "GO:1990745"
}